12-hydroxyheptadecatrienoic acid synthase activity [GO:0036134] (molecular function) Also known as: prostaglandin H2 degradation activity Relationships: is_a oxidoreductase activity, acting on the CH-CH group of donors, NAD or NADP as acceptor [GO:0016628] Definition: Catalysis of the reaction: prostaglandin H2 = 12-hydroxyheptadecatrienoic acid (HHT) + malonaldehyde (MDA). References: PMID:11297515 Sources: GOC:mw